positive regulation of nematode larval development, heterochronic [GO:0090445] (biological process) Relationships: is a type of positive regulation of development, heterochronic [GO:0045962]; is a type of positive regulation of nematode larval development [GO:0061063]; is a type of regulation of nematode larval development, heterochronic [GO:0090444] Definition: Any process that modulates the consistent predetermined time point at which a nematode larva progresses from an initial condition to a later condition and increases the rate at which this time point is reached. References: PMID:17550772